{
  "term_id": "GO:0000981",
  "gene_name": "POU domain, class 5, transcription factor 1",
  "gene": "UniProtKB:Q01860",
  "gene_symbol": "POU5F1",
  "term_label": "DNA-binding transcription factor activity, RNA polymerase II-specific"
}